N6-(1,2-dicarboxyethyl)AMP AMP-lyase (fumarate-forming) activity [GO:0004018] (MF) Sources: RHEA:16853 Definition: Catalysis of the reaction: N6-(1,2-dicarboxyethyl)AMP = fumarate + AMP. Relationships: is a type of amidine-lyase activity [GO:0016842] Also known as: adenylosuccinase activity, adenylosuccinate lyase activity, succino AMP-lyase activity, 6-N-(1,2-dicarboxyethyl)AMP AMP-lyase activity, N6-(1,2-dicarboxyethyl)AMP AMP-lyase activity